phenylpropanoyltransferase activity [GO:0102922] (molecular function) Sources: RHEA:42488 Relationships: is a type of GO:0016747 Definition: Catalysis of the reaction: (3R)-3-amino-3-phenylpropanoyl-CoA + baccatin III = 3'-N-debenzoyl-2'-deoxytaxol + CoA.